{
  "gene": "UniProtKB:Q9UK05",
  "gene_name": "Growth_differentiation factor 2",
  "gene_symbol": "GDF2",
  "term_id": "GO:0001938",
  "term_label": "positive regulation of endothelial cell proliferation"
}